regulation of ubiquitin protein ligase activity [GO:1904666] (biological process) References: PMID:10921876, PMID:26216882 Sources: GOC:TermGenie, GOC:dph, GOC:vw, GO_REF:0000059 Definition: Any process that modulates the frequency, rate or extent of ubiquitin protein ligase activity. Also known as: regulation of protein ubiquitination activity, regulation of ubiquitin ligase activity, regulation of APC-fizzy related complex activity, regulation of E3 Relationships: is a type of regulation of ubiquitin-protein transferase activity [GO:0051438]; RO_0002211 ubiquitin protein ligase activity [GO:0061630] Subtypes: negative regulation of ubiquitin protein ligase activity [GO:1904667], positive regulation of ubiquitin protein ligase activity [GO:1904668]